premeiotic DNA replication termination [GO:1902978] (biological process) Definition: Any DNA replication termination involved in meiotic cell cycle DNA replication. Sources: GOC:TermGenie, GO_REF:0000060 Also known as: DNA replication termination involved in meiotic DNA replication, DNA replication termination involved in meiotic cell cycle DNA replication Relationships: is a type of GO:1902317; is a type of meiotic cell cycle process [GO:1903046]; is part of premeiotic DNA replication [GO:0006279]